nuclear export [GO:0051168] (biological process) Definition: The directed movement of substances out of the nucleus. Sources: GOC:ai Also known as: export from nucleus, nucleus export, substance nuclear export Relationships: is a type of nucleocytoplasmic transport [GO:0006913] Subtypes: ribosomal subunit export from nucleus [GO:0000054], RNA export from nucleus [GO:0006405], protein export from nucleus [GO:0006611], nuclear envelope budding [GO:0140591]